{
  "term_id": "UNKNOWN:0002",
  "gene_symbol": "TEX9",
  "gene": "UniProtKB:Q8N6V9",
  "term_label": "Unknown biological process",
  "gene_name": "Testis-expressed protein 9"
}